{
  "gene_name": "Mitochondrial ubiquitin ligase activator of NFKB 1",
  "gene": "UniProtKB:Q969V5",
  "term_id": "GO:0050821",
  "term_label": "protein stabilization",
  "gene_symbol": "MUL1"
}